UDP-galactose transmembrane import into Golgi lumen [GO:0097624] (biological process) References: PMID:11378902 Sources: GOC:vw Also known as: UDP-galactose import into Golgi lumen Definition: The directed movement of UDP-galactose into the Golgi lumen across the Golgi membrane. Relationships: is a type of UDP-galactose transmembrane transport [GO:0072334]